{
  "gene": "UniProtKB:P04054",
  "term_label": "phosphatidylglycerol metabolic process",
  "gene_name": "Phospholipase A2",
  "gene_symbol": "PLA2G1B",
  "term_id": "GO:0046471"
}